mitotic cell cycle G1 arrest in response to pheromone [GO:0000751] (biological process) Definition: The cell cycle regulatory process in which the mitotic cell cycle is halted during G1 as a result of a pheromone stimulus. An example of this process is found in Saccharomyces cerevisiae. Also known as: cell cycle arrest in response to pheromone Relationships: is a type of negative regulation of mitotic cell cycle [GO:0045930]; is part of response to pheromone triggering conjugation with cellular fusion [GO:0000749] Sources: GOC:clt, GOC:dph, GOC:mah, GOC:tb